{
  "gene_symbol": "FAM27C",
  "gene": "UniProtKB:Q5VT28",
  "term_id": "UNKNOWN:0003",
  "gene_name": "Protein FAM27A_B_C",
  "term_label": "Unknown cellular component"
}